{
  "term_label": "Unknown molecular function",
  "gene_symbol": "A0A8Q3SIZ7",
  "gene": "UniProtKB:A0A8Q3SIZ7",
  "term_id": "UNKNOWN:0001",
  "gene_name": "Uncharacterized protein"
}